{
  "gene": "UniProtKB:Q9Y2Y8",
  "gene_name": "Proteoglycan 3",
  "term_id": "UNKNOWN:0002",
  "term_label": "Unknown biological process",
  "gene_symbol": "PRG3"
}